cyclic purine nucleotide metabolic process [GO:0052652] (biological process) Relationships: is a type of purine nucleotide metabolic process [GO:0006163]; is a type of cyclic nucleotide metabolic process [GO:0009187] Also known as: cyclic purine nucleotide metabolism Definition: The chemical reactions and pathways involving a cyclic nucleotide, a nucleotide in which the phosphate group is in diester linkage to two positions on the sugar residue and the base is a purine. References: PMID:23911318 Subtypes: cAMP metabolic process [GO:0046058], cGMP metabolic process [GO:0046068]